{
  "term_label": "Unknown cellular component",
  "term_id": "UNKNOWN:0003",
  "gene": "UniProtKB:P48775",
  "gene_name": "Tryptophan 2,3-dioxygenase",
  "gene_symbol": "TDO2"
}